positive regulation of arachidonate secretion [GO:0090238] (biological process) Sources: GOC:BHF, GOC:dph, GOC:tb Definition: Any process that increases the rate, frequency, or extent of arachidonic acid secretion, the controlled release of arachidonic acid from a cell or a tissue. Relationships: is a type of GO:0032305; is a type of regulation of arachidonate secretion [GO:0090237]; positively regulates GO:0050482 Also known as: positive regulation of arachidonic acid secretion